{
  "gene_symbol": "ZNF674",
  "term_label": "DNA-binding transcription factor activity, RNA polymerase II-specific",
  "term_id": "GO:0000981",
  "gene_name": "Zinc finger protein 674",
  "gene": "UniProtKB:Q2M3X9"
}